{
  "term_label": "Unknown molecular function",
  "gene_symbol": "ANKRD36BP1",
  "gene_name": "Putative ankyrin repeat domain-containing protein 26-like 1",
  "term_id": "UNKNOWN:0001",
  "gene": "UniProtKB:Q96IX9"
}